{
  "gene_symbol": "RNF208",
  "gene_name": "RING finger protein 208",
  "term_label": "Unknown cellular component",
  "gene": "UniProtKB:Q9H0X6",
  "term_id": "UNKNOWN:0003"
}